{
  "term_label": "Unknown molecular function",
  "gene_name": "Carcinoembryonic antigen-related cell adhesion molecule 21",
  "term_id": "UNKNOWN:0001",
  "gene": "UniProtKB:Q3KPI0",
  "gene_symbol": "CEACAM21"
}